negative regulation of cellular extravasation [GO:0002692] (biological process) Definition: Any process that stops, prevents, or reduces the frequency, rate, or extent of cellular extravasation. Sources: GOC:add Also known as: down regulation of cellular extravasation, down-regulation of cellular extravasation, downregulation of cellular extravasation, inhibition of cellular extravasation Relationships: is a type of negative regulation of leukocyte migration [GO:0002686]; is a type of GO:0002691; negatively regulates cellular extravasation [GO:0045123] Subtypes: negative regulation of leukocyte tethering or rolling [GO:1903237], GO:2000390, negative regulation of T cell extravasation [GO:2000408], GO:2000420, GO:2000438